positive regulation of synaptic vesicle lumen acidification [GO:1901548] (biological process) Sources: GOC:TermGenie Also known as: positive regulation of proton loading, positive regulation of synaptic vesicle lumen pH reduction, up regulation of synaptic vesicle lumen acidification, up regulation of synaptic vesicle lumen pH reduction, up-regulation of synaptic vesicle lumen acidification, up-regulation of synaptic vesicle lumen pH reduction, upregulation of synaptic vesicle lumen acidification, upregulation of synaptic vesicle lumen pH reduction, activation of synaptic vesicle lumen acidification, activation of synaptic vesicle lumen pH reduction Definition: Any process that activates or increases the frequency, rate or extent of synaptic vesicle lumen acidification. Relationships: is a type of GO:1901546; is a type of positive regulation of cation transmembrane transport [GO:1904064]; positively regulates synaptic vesicle lumen acidification [GO:0097401]